{
  "term_id": "GO:0016773",
  "gene_symbol": "POMK",
  "gene_name": "Protein O-mannose kinase",
  "term_label": "phosphotransferase activity, alcohol group as acceptor",
  "gene": "UniProtKB:Q9H5K3"
}